positive regulation of nucleosome disassembly [GO:0140887] (biological process) Definition: Any process that activates or increases the frequency, rate or extent of the controlled breakdown of nucleosomes, the beadlike structural units of eukaryotic chromatin composed of histones and DNA. References: PMID:34471130, PMID:35308047 Relationships: is a type of GO:0031334; is a type of positive regulation of chromatin organization [GO:1905269]; RO_0002213 nucleosome assembly [GO:0006334]